response to molecule of bacterial origin [GO:0002237] (biological process) Definition: Any process that results in a change in state or activity of an organism (in terms of movement, secretion, enzyme production, gene expression, etc.) as a result of a stimulus by molecules of bacterial origin such as peptides derived from bacterial flagellin. Sources: GOC:rl, GOC:sm Also known as: response to bacteria associated molecule, response to bacterial associated molecule, response to bacterium associated molecule Relationships: is a type of response to external biotic stimulus [GO:0043207]; is part of response to bacterium [GO:0009617] Subtypes: detection of molecule of bacterial origin [GO:0032490], response to bacterial lipoprotein [GO:0032493], response to peptidoglycan [GO:0032494], response to lipopolysaccharide [GO:0032496], GO:0070391, GO:0071219